{
  "term_id": "UNKNOWN:0001",
  "gene": "UniProtKB:Q9NRJ4",
  "term_label": "Unknown molecular function",
  "gene_symbol": "TULP4",
  "gene_name": "Tubby-related protein 4"
}